L-glutamate:proton antiporter activity [GO:0106421] (molecular function) References: PMID:29273736 Relationships: is a type of L-glutamate transmembrane transporter activity [GO:0005313]; is a type of proton transmembrane transporter activity [GO:0015078]; is a type of amino acid:monoatomic cation antiporter activity [GO:0140848] Subtypes: GO:0000515 Definition: Enables the transfer of a solute or solutes from one side of a membrane to the other according to the reaction: L-glutamate(out) + H+(in) = L-glutamate(in) + H+(out).